D-xylose reductase (NADPH) activity [GO:0032866] (molecular function) Also known as: D-xylose reductase activity, xylose reductase activity, D-xylose:NADP reductase activity Relationships: is a type of aldose reductase (NADPH) activity [GO:0004032] Definition: Catalysis of the reaction: D-xylitol + NADP+ = D-xylose + NADPH + H+. References: PMID:12724380, PMID:15184173 Sources: RHEA:27445